{
  "gene_symbol": "DLX1",
  "gene_name": "Homeobox protein DLX-1",
  "gene": "UniProtKB:P56177",
  "term_label": "cell differentiation",
  "term_id": "GO:0030154"
}